{
  "gene": "UniProtKB:H3BQL2",
  "gene_symbol": "GOLGA8T",
  "term_id": "GO:0007030",
  "term_label": "Golgi organization",
  "gene_name": "Golgin subfamily A member 8T"
}